cell adhesive protein binding involved in SA cardiac muscle cell-atrial cardiac muscle cell communication [GO:0086085] (molecular function) Sources: GOC:BHF, GOC:mtg_cardiac_conduct_nov11 Also known as: cell adhesive protein binding involved in SA cardiomyocyte-atrial cardiomyocyte communication Definition: Binding to a protein or protein complex that results in the connection of an SA cardiomyocyte with an atrial cardiomyocyte and contributes to the communication between the two cells. Relationships: is_a protein binding involved in heterotypic cell-cell adhesion [GO:0086080]; is part of SA node cell-atrial cardiac muscle cell adhesion involved in cell communication [GO:0086022]